ergosterol O-acyltransferase activity [GO:0034737] (molecular function) Relationships: is a type of GO:0004772 Sources: GOC:mah Definition: Catalysis of the reaction: acyl-CoA + ergosterol = CoA + ergosterol ester.